{
  "term_label": "double-strand break repair via break-induced replication",
  "gene_name": "DNA replication complex GINS protein PSF2",
  "term_id": "GO:0000727",
  "gene_symbol": "GINS2",
  "gene": "UniProtKB:Q9Y248"
}